{
  "gene_name": "Cytochrome b5",
  "gene_symbol": "CYB5A",
  "gene": "UniProtKB:P00167",
  "term_id": "GO:0020037",
  "term_label": "heme binding"
}